{
  "term_label": "DNA-directed DNA polymerase activity",
  "gene_name": "DNA-directed DNA_RNA polymerase mu",
  "gene": "UniProtKB:Q9NP87",
  "term_id": "GO:0003887",
  "gene_symbol": "POLM"
}